{
  "gene_symbol": "CCDC117",
  "term_id": "UNKNOWN:0002",
  "gene_name": "Coiled-coil domain-containing protein 117",
  "term_label": "Unknown biological process",
  "gene": "UniProtKB:Q8IWD4"
}